{
  "term_id": "GO:0008083",
  "gene_symbol": "CSF3",
  "gene": "UniProtKB:P09919",
  "term_label": "growth factor activity",
  "gene_name": "Granulocyte colony-stimulating factor"
}